{
  "gene_symbol": "SLC26A10P",
  "gene": "UniProtKB:Q8NG04",
  "term_label": "sulfate transmembrane transport",
  "term_id": "GO:1902358",
  "gene_name": "Putative solute carrier family 26 member 10P"
}